positive regulation of gliogenesis [GO:0014015] (biological process) Relationships: is a type of regulation of gliogenesis [GO:0014013]; is a type of GO:0050769; positively regulates gliogenesis [GO:0042063] Subtypes: positive regulation of glial cell differentiation [GO:0045687], positive regulation of glial cell proliferation [GO:0060252], GO:0070447 Also known as: up regulation of gliogenesis, up-regulation of gliogenesis, upregulation of gliogenesis, activation of gliogenesis, stimulation of gliogenesis Definition: Any process that activates or increases the frequency, rate or extent of gliogenesis, the formation of mature glia. Sources: GOC:ef